positive regulation of cell proliferation in midbrain [GO:1904935] (biological process) Also known as: positive regulation of cell proliferation in mesencephalon, up regulation of cell proliferation in mesencephalon, up regulation of cell proliferation in midbrain, up-regulation of cell proliferation in mesencephalon, up-regulation of cell proliferation in midbrain, upregulation of cell proliferation in mesencephalon, upregulation of cell proliferation in midbrain, activation of cell proliferation in mesencephalon, activation of cell proliferation in midbrain, activation of mesencepahalic cell proliferation, positive regulation of mesencepahalic cell proliferation, up regulation of mesencepahalic cell proliferation, up-regulation of mesencepahalic cell proliferation, upregulation of mesencepahalic cell proliferation References: PMID:24431302 Sources: GOC:PARL, GOC:TermGenie, GOC:bf, GO_REF:0000058 Definition: Any process that activates or increases the frequency, rate or extent of cell proliferation in midbrain. Relationships: is a type of regulation of cell proliferation in midbrain [GO:1904933]; is a type of positive regulation of neural precursor cell proliferation [GO:2000179]; positively regulates cell proliferation in midbrain [GO:0033278]